{
  "gene_symbol": "TRAPPC6B",
  "term_id": "GO:0005802",
  "term_label": "trans-Golgi network",
  "gene_name": "Trafficking protein particle complex subunit 6B",
  "gene": "UniProtKB:Q86SZ2"
}